{
  "gene_symbol": "SNU13",
  "term_label": "nucleolus",
  "term_id": "GO:0005730",
  "gene": "UniProtKB:P55769",
  "gene_name": "NHP2-like protein 1"
}